{
  "term_id": "GO:0030036",
  "gene_name": "Formin-2",
  "gene": "UniProtKB:Q9NZ56",
  "term_label": "actin cytoskeleton organization",
  "gene_symbol": "FMN2"
}